{
  "gene_name": "Olfactory receptor 52I2",
  "gene": "UniProtKB:Q8NH67",
  "term_label": "Unknown biological process",
  "term_id": "UNKNOWN:0002",
  "gene_symbol": "OR52I2"
}